{
  "term_label": "membrane",
  "gene": "UniProtKB:Q92544",
  "gene_symbol": "TM9SF4",
  "gene_name": "Transmembrane 9 superfamily member 4",
  "term_id": "GO:0016020"
}